N-feruloylglycine deacylase activity [GO:0050128] (molecular function) Definition: Catalysis of the reaction: N-feruloylglycine + H2O = ferulate + glycine. Sources: EC:3.5.1.71, RHEA:10484 Also known as: N-feruloylglycine amidohydrolase activity, N-feruloylglycine hydrolase activity Relationships: is a type of hydrolase activity, acting on carbon-nitrogen (but not peptide) bonds, in linear amides [GO:0016811]